poly(U)-specific exoribonuclease activity, producing 3' uridine cyclic phosphate ends [GO:1990838] (molecular function) Relationships: is a type of 3'-5'-RNA exonuclease activity [GO:0000175] Definition: Catalysis of the reaction: a 3'-end uridylyl-uridine-RNA = a 3'-end 2',3'-cyclophospho-uridine-RNA + uridine. References: PMID:23022480 Sources: RHEA:46052